organic phosphonate metabolic process [GO:0019634] (biological process) Also known as: phosphonate metabolism, organophosphonate metabolic process Definition: The chemical reactions and pathways involving phosphonates, any organic compounds containing one or more C-PO(OH)2 or C-PO(OR)2 (with R=alkyl, aryl) groups. Metabolism of phosphonic acid itself, an inorganic compound without the biochemically relevant C-P bond, is not included. Sources: GOC:js, ISBN:0721662544 Relationships: is a type of phosphorus metabolic process [GO:0006793]; is a type of GO:0043436 Subtypes: organic phosphonate catabolic process [GO:0019700], organic phosphonate biosynthetic process [GO:0032923]